{
  "gene_name": "Peptidyl-prolyl cis-trans isomerase G",
  "term_label": "peptidyl-prolyl cis-trans isomerase activity",
  "gene": "UniProtKB:Q13427",
  "gene_symbol": "PPIG",
  "term_id": "GO:0003755"
}